{
  "gene": "UniProtKB:Q7Z569",
  "term_id": "GO:0016567",
  "term_label": "protein ubiquitination",
  "gene_name": "BRCA1-associated protein",
  "gene_symbol": "BRAP"
}